{
  "term_label": "melanocortin receptor activity",
  "gene_name": "Melanocortin receptor 5",
  "term_id": "GO:0004977",
  "gene": "UniProtKB:P33032",
  "gene_symbol": "MC5R"
}